{
  "term_id": "GO:0003684",
  "term_label": "damaged DNA binding",
  "gene_symbol": "XPA",
  "gene_name": "DNA repair protein complementing XP-A cells",
  "gene": "UniProtKB:P23025"
}